{
  "gene": "UniProtKB:Q6NW40",
  "gene_symbol": "RGMB",
  "gene_name": "Repulsive guidance molecule B",
  "term_label": "coreceptor activity",
  "term_id": "GO:0015026"
}